{
  "gene_symbol": "DRAP1",
  "term_label": "transcription by RNA polymerase II",
  "gene": "UniProtKB:Q14919",
  "term_id": "GO:0006366",
  "gene_name": "Dr1-associated corepressor"
}